nitrile metabolic process [GO:0050898] (biological process) Also known as: nitrile metabolism Definition: The chemical reactions and pathways involving nitriles, an organic compound containing trivalent nitrogen attached to one carbon atom. The nitriles are named with reference to the acids produced by their decomposition; for example, hydrocyanic acid is formic nitrile, and methyl cyanide is acetic nitrile. Subtypes: benzonitrile metabolic process [GO:0018876], bromoxynil metabolic process [GO:0018881], cyanamide metabolic process [GO:0018890], nitrile catabolic process [GO:0050899], nitrile biosynthetic process [GO:0080028], 7-cyano-7-deazaguanine metabolic process [GO:0097287] References: PMID:18987211 Relationships: is_a metabolic process [GO:0008152]